{
  "gene": "UniProtKB:P35789",
  "term_label": "regulation of transcription by RNA polymerase II",
  "term_id": "GO:0006357",
  "gene_symbol": "ZNF93",
  "gene_name": "Zinc finger protein 93"
}